{
  "term_label": "proteolysis",
  "term_id": "GO:0006508",
  "gene": "UniProtKB:P55786",
  "gene_name": "Puromycin-sensitive aminopeptidase",
  "gene_symbol": "NPEPPS"
}